cytoplasmic ribonucleoprotein granule [GO:0036464] (cellular component) References: PMID:15121898 Sources: GOC:PARL, GOC:bf Subtypes: GO:0000932, cytoplasmic stress granule [GO:0010494], GO:0033391, P granule [GO:0043186], GO:0070725, cytoplasmic U snRNP body [GO:0071254], neuronal ribonucleoprotein granule [GO:0071598], Z granule [GO:0120279], TIS granule [GO:0140363], GO:0140364, RNP body [GO:0140365], mutator focus [GO:1990633] Relationships: is a type of ribonucleoprotein granule [GO:0035770]; is part of cytoplasm [GO:0005737] Also known as: Staufen granule Definition: A ribonucleoprotein granule located in the cytoplasm.